{
  "gene": "UniProtKB:Q13370",
  "term_label": "negative regulation of cAMP/PKA signal transduction",
  "gene_symbol": "PDE3B",
  "term_id": "GO:0141162",
  "gene_name": "cGMP-inhibited 3',5'-cyclic phosphodiesterase 3B"
}